{
  "gene": "UniProtKB:Q5TA78",
  "gene_symbol": "LCE4A",
  "term_id": "UNKNOWN:0001",
  "term_label": "Unknown molecular function",
  "gene_name": "Late cornified envelope protein 4A"
}